{
  "term_id": "GO:0001889",
  "gene": "UniProtKB:P55789",
  "gene_name": "FAD-linked sulfhydryl oxidase ALR",
  "term_label": "liver development",
  "gene_symbol": "GFER"
}